{
  "gene_name": "Putative uncharacterized protein RUSC1-AS1",
  "gene_symbol": "RUSC1-AS1",
  "term_id": "UNKNOWN:0001",
  "term_label": "Unknown molecular function",
  "gene": "UniProtKB:Q66K80"
}